corticotropin-releasing hormone receptor 1 binding [GO:0051430] (molecular function) Relationships: is a type of corticotropin-releasing hormone receptor binding [GO:0051429] Also known as: CRHR1 binding, type 1 corticotropin releasing factor receptor binding, type 1 corticotropin-releasing factor receptor binding, type 1 corticotropin releasing factor receptor ligand References: PMID:15134857 Definition: Binding to a corticotropin-releasing hormone receptor 1 (CRHR1). CRHR1 is the major subtype in the pituitary corticotroph, and mediates the stimulatory actions of corticotropin-releasing hormone on corticotropin hormone secretion. CRHR1 are also located in cortical areas of the brain, cerebellum and limbic system.